{
  "gene": "UniProtKB:Q9NZJ9",
  "term_label": "bis(5'-adenosyl)-hexaphosphatase activity",
  "gene_symbol": "NUDT4",
  "gene_name": "Diphosphoinositol polyphosphate phosphohydrolase 2",
  "term_id": "GO:0034431"
}